{
  "term_id": "GO:0045271",
  "term_label": "respiratory chain complex I",
  "gene_symbol": "MT-ND4L",
  "gene": "UniProtKB:P03901",
  "gene_name": "NADH-ubiquinone oxidoreductase chain 4L"
}